{
  "gene_name": "Transmembrane protein 186",
  "term_label": "mitochondrion",
  "term_id": "GO:0005739",
  "gene_symbol": "TMEM186",
  "gene": "UniProtKB:Q96B77"
}